regulation of glutamate metabolic process [GO:2000211] (biological process) Also known as: regulation of glutamate metabolism, regulation of glutamic acid metabolic process, regulation of glutamic acid metabolism Sources: GOC:sl Subtypes: regulation of tetrapyrrole biosynthetic process from glutamate [GO:1901410], negative regulation of glutamate metabolic process [GO:2000212], regulation of L-proline catabolic process to L-glutamate [GO:2001156], regulation of ammonia assimilation cycle [GO:2001248] Definition: Any process that modulates the frequency, rate or extent of glutamate metabolic process. Relationships: is_a regulation of amino acid metabolic process [GO:0006521]; is a type of regulation of small molecule metabolic process [GO:0062012]; regulates GO:0006536